{
  "gene_symbol": "ZNF573",
  "gene": "UniProtKB:Q86YE8",
  "term_id": "GO:0000981",
  "term_label": "DNA-binding transcription factor activity, RNA polymerase II-specific",
  "gene_name": "Zinc finger protein 573"
}